{
  "term_id": "GO:0004175",
  "term_label": "endopeptidase activity",
  "gene": "UniProtKB:P28065",
  "gene_name": "Proteasome subunit beta type-9",
  "gene_symbol": "PSMB9"
}